{
  "term_label": "cytosol",
  "term_id": "GO:0005829",
  "gene_symbol": "RIN1",
  "gene_name": "Ras and Rab interactor 1",
  "gene": "UniProtKB:Q13671"
}